{
  "gene_name": "Mothers against decapentaplegic homolog 5",
  "term_id": "GO:0000978",
  "gene_symbol": "SMAD5",
  "term_label": "RNA polymerase II cis-regulatory region sequence-specific DNA binding",
  "gene": "UniProtKB:Q99717"
}